{
  "gene_name": "Guanine nucleotide-binding protein G(s) subunit alpha isoforms XLas",
  "gene_symbol": "GNAS",
  "term_label": "cytoplasm",
  "term_id": "GO:0005737",
  "gene": "UniProtKB:Q5JWF2"
}